galactosylceramide catabolic process [GO:0006683] (biological process) Definition: The chemical reactions and pathways resulting in the breakdown of galactosylceramides, any compound formed by the replacement of the glycosidic hydroxyl group of a cyclic form of galactose by a ceramide group. Sources: GOC:ai Also known as: galactosylceramide breakdown, galactosylceramide catabolism, galactosylceramide degradation Relationships: is a type of GO:0006681; is a type of galactolipid catabolic process [GO:0019376]; is a type of GO:0046477